isopentenyl adenine biosynthetic process [GO:0034265] (biological process) References: PMID:18216168 Sources: GOC:mah Also known as: isopentenyl adenine anabolism, isopentenyl adenine biosynthesis, isopentenyl adenine formation, isopentenyl adenine synthesis, isopentenyladenine biosynthetic process Relationships: is a type of cytokinin biosynthetic process [GO:0009691]; is a type of purine-containing compound biosynthetic process [GO:0072522] Definition: The chemical reactions and pathways resulting in the formation of the cytokinin 6-isopentenyladenine.